{
  "gene_name": "Protein Mis18-beta",
  "gene": "UniProtKB:O43482",
  "term_id": "UNKNOWN:0001",
  "term_label": "Unknown molecular function",
  "gene_symbol": "OIP5"
}